{
  "gene_name": "Probable phospholipid-transporting ATPase IM",
  "term_id": "GO:0005886",
  "gene": "UniProtKB:Q8TF62",
  "term_label": "plasma membrane",
  "gene_symbol": "ATP8B4"
}